{
  "term_label": "structural constituent of muscle",
  "gene_name": "Myosin-binding protein C, slow-type",
  "term_id": "GO:0008307",
  "gene_symbol": "MYBPC1",
  "gene": "UniProtKB:Q00872"
}